{
  "term_id": "UNKNOWN:0001",
  "gene_symbol": "DSCR10",
  "gene_name": "Down syndrome critical region protein 10",
  "gene": "UniProtKB:P59022",
  "term_label": "Unknown molecular function"
}